{
  "term_id": "GO:0005794",
  "gene_name": "Solute carrier family 35 member E2A",
  "gene": "UniProtKB:P0CK97",
  "term_label": "Golgi apparatus",
  "gene_symbol": "SLC35E2A"
}